taxadiene synthase activity [GO:0050553] (molecular function) Relationships: is a type of carbon-oxygen lyase activity, acting on phosphates [GO:0016838] Definition: Catalysis of the reaction: all-trans-geranylgeranyl diphosphate = diphosphate + taxa-4,11-diene. Sources: EC:4.2.3.17, RHEA:20912 Also known as: geranylgeranyl-diphosphate diphosphate-lyase (cyclizing, taxa-4,11-diene-forming), geranylgeranyl-diphosphate diphosphate-lyase (cyclizing, taxadiene-forming), taxa-4(5),11(12)-diene synthase activity